{
  "gene_symbol": "BICD2",
  "gene_name": "Protein bicaudal D homolog 2",
  "term_id": "GO:0051959",
  "gene": "UniProtKB:Q8TD16",
  "term_label": "dynein light intermediate chain binding"
}